{
  "gene_name": "Alpha-actinin-3",
  "term_id": "GO:0030054",
  "gene_symbol": "ACTN3",
  "term_label": "cell junction",
  "gene": "UniProtKB:Q08043"
}